{
  "gene_name": "Aspartate--tRNA ligase, cytoplasmic",
  "term_label": "aspartate-tRNA ligase activity",
  "term_id": "GO:0004815",
  "gene": "UniProtKB:P14868",
  "gene_symbol": "DARS1"
}